{
  "term_id": "GO:0045109",
  "gene_name": "Alpha-internexin",
  "gene": "UniProtKB:Q16352",
  "term_label": "intermediate filament organization",
  "gene_symbol": "INA"
}